{
  "term_label": "extracellular space",
  "gene_symbol": "CTSW",
  "term_id": "GO:0005615",
  "gene": "UniProtKB:P56202",
  "gene_name": "Cathepsin W"
}